L-histidine catabolic process [GO:0006548] (biological process) Subtypes: L-histidine catabolic process to glutamate and formamide [GO:0019556], L-histidine catabolic process to glutamate and formate [GO:0019557], L-histidine catabolic process to 2-oxoglutarate [GO:0019558], L-histidine catabolic process to imidazol-5-yl-lactate [GO:0019559], L-histidine catabolic process to hydantoin-5-propionate [GO:0019560] Definition: The chemical reactions and pathways resulting in the breakdown of L-histidine, 2-amino-3-(1H-imidazol-4-yl)propanoic acid. Sources: GOC:go_curators Relationships: is a type of GO:0006547; is a type of aromatic amino acid family catabolic process [GO:0009074]; is a type of imidazole-containing compound catabolic process [GO:0052805]; is a type of L-amino acid catabolic process [GO:0170035]; is a type of proteinogenic amino acid catabolic process [GO:0170040] Also known as: histidine catabolic process, histidine breakdown, histidine catabolism, histidine degradation